glial cell projection elongation involved in axon ensheathment [GO:0106092] (biological process) Relationships: is a type of axon ensheathment [GO:0008366]; is a type of glial cell projection elongation [GO:0106091] Definition: The extension of a glial cell process or projection to wrap around an axon. References: PMID:27131624 Sources: GOC:ha